histone H4K20me1 reader activity [GO:0140117] (molecular function) References: PMID:19494831 Also known as: H4K20me1 modified histone binding Definition: A histone reader that recognizes a histone H4 monomethylated at lysine 20. Note: Note that the residue position corresponds to the canonical human H4 histone (UniProtKB:P02309); this residue is conserved across all eukaryotes. Note that the initiation methionine is cleaved, so the first residue is S1. Relationships: is_a histone H4 reader activity [GO:0140008]